{
  "gene_name": "Coiled-coil domain-containing protein 180",
  "term_label": "Unknown biological process",
  "gene_symbol": "CCDC180",
  "term_id": "UNKNOWN:0002",
  "gene": "UniProtKB:Q9P1Z9"
}